{
  "gene": "UniProtKB:O15027",
  "gene_symbol": "SEC16A",
  "term_id": "GO:0043495",
  "gene_name": "Protein transport protein Sec16A",
  "term_label": "protein-membrane adaptor activity"
}